{
  "gene_name": "Trafficking kinesin-binding protein 2",
  "gene_symbol": "TRAK2",
  "gene": "UniProtKB:O60296",
  "term_label": "mitochondrion",
  "term_id": "GO:0005739"
}